{
  "term_id": "GO:0016412",
  "gene_name": "Ghrelin O-acyltransferase",
  "gene": "UniProtKB:Q96T53",
  "gene_symbol": "MBOAT4",
  "term_label": "serine O-acyltransferase activity"
}